positive regulation of calcium ion import into sarcoplasmic reticulum [GO:1902082] (biological process) Definition: Any process that activates or increases the frequency, rate or extent of calcium ion import into sarcoplasmic reticulum. References: PMID:8349590 Sources: GOC:BHF, GOC:TermGenie, GOC:rl Relationships: is a type of GO:0032388; is a type of positive regulation of calcium ion transport [GO:0051928]; is a type of GO:1902080; positively regulates calcium ion import into sarcoplasmic reticulum [GO:1990036] Also known as: up regulation of calcium ion import into sarcoplasmic reticulum, up-regulation of calcium ion import into sarcoplasmic reticulum, upregulation of calcium ion import into sarcoplasmic reticulum, activation of calcium ion import into sarcoplasmic reticulum